gamma-tubulin complex [GO:0000930] (cellular component) Definition: A multiprotein complex composed of gamma-tubulin and other non-tubulin proteins. Gamma-tubulin complexes are localized to microtubule organizing centers, and play an important role in the nucleation of microtubules. The number and complexity of non-tubulin proteins associated with these complexes varies between species. Subtypes: gamma-tubulin ring complex [GO:0000931], GO:0008275 Relationships: is a type of protein-containing complex [GO:0032991]; is part of microtubule organizing center [GO:0005815] References: PMID:12134075 Sources: GOC:clt